{
  "gene_symbol": "SNCB",
  "term_label": "cuprous ion binding",
  "gene_name": "Beta-synuclein",
  "gene": "UniProtKB:Q16143",
  "term_id": "GO:1903136"
}